{
  "gene_symbol": "GCKR",
  "term_label": "glucose sensor activity",
  "term_id": "GO:0141089",
  "gene_name": "Glucokinase regulatory protein",
  "gene": "UniProtKB:Q14397"
}